succinate transmembrane transport [GO:0071422] (biological process) Subtypes: succinate import across plasma membrane [GO:0098720] Note: Note that this term is not intended for use in annotating lateral movement within membranes. Definition: The process in which succinate is transported across a membrane. Also known as: succinate membrane transport, transmembrane succinate transport Sources: GOC:mah Relationships: is a type of succinate transport [GO:0015744]; is a type of carboxylic acid transmembrane transport [GO:1905039]